tumor necrosis factor superfamily cytokine production [GO:0071706] (biological process) Regulation: regulated by GO:1903555; negatively regulated by negative regulation of tumor necrosis factor superfamily cytokine production [GO:1903556]; positively regulated by positive regulation of tumor necrosis factor superfamily cytokine production [GO:1903557] Definition: The appearance of any member of the TNF superfamily due to biosynthesis or secretion following a cellular stimulus, resulting in an increase in its intracellular or extracellular levels. Also known as: TNFSF cytokine production, TNF superfamily production Relationships: is a type of GO:0001816 Note: Note that this term is in the subset of terms that should not be used for direct gene product annotation. Instead, select one of the 'regulation' children terms. Subtypes: GO:0032639, tumor necrosis factor production [GO:0032640], lymphotoxin A production [GO:0032641], tumor necrosis factor (ligand) superfamily member 11 production [GO:0072535] Sources: GOC:add